{
  "term_id": "GO:0005654",
  "gene": "UniProtKB:Q6IN85",
  "gene_symbol": "PPP4R3A",
  "gene_name": "Serine_threonine-protein phosphatase 4 regulatory subunit 3A",
  "term_label": "nucleoplasm"
}